{
  "gene": "UniProtKB:Q86UW2",
  "gene_symbol": "SLC51B",
  "gene_name": "Organic solute transporter subunit beta",
  "term_id": "GO:0015125",
  "term_label": "bile acid transmembrane transporter activity"
}